{
  "gene": "UniProtKB:Q8IWA5",
  "term_label": "membrane",
  "gene_symbol": "SLC44A2",
  "gene_name": "Choline transporter-like protein 2",
  "term_id": "GO:0016020"
}